negative regulation of cardiac muscle cell contraction [GO:0106135] (biological process) Definition: Any process that stops, prevents, or reduces the frequency, rate or extent of cardiac muscle cell contraction. Subtypes: negative regulation of ventricular cardiac muscle cell action potential [GO:1903946], negative regulation of atrial cardiac muscle cell action potential [GO:1903948] References: PMID:19525381 Relationships: is a type of GO:0048523; is a type of negative regulation of cardiac muscle contraction [GO:0055118]; is a type of regulation of cardiac muscle cell contraction [GO:0086004]; negatively regulates cardiac muscle cell contraction [GO:0086003]